{
  "gene": "UniProtKB:Q969Y2",
  "gene_symbol": "GTPBP3",
  "gene_name": "tRNA modification GTPase GTPBP3, mitochondrial",
  "term_label": "mitochondrion",
  "term_id": "GO:0005739"
}